{
  "term_id": "GO:0005615",
  "term_label": "extracellular space",
  "gene_symbol": "CCL8",
  "gene": "UniProtKB:P80075",
  "gene_name": "C-C motif chemokine 8"
}